{
  "gene": "UniProtKB:Q08999",
  "term_id": "GO:0030154",
  "gene_symbol": "RBL2",
  "term_label": "cell differentiation",
  "gene_name": "Retinoblastoma-like protein 2"
}